{
  "term_label": "signaling receptor binding",
  "gene_symbol": "PEX14",
  "gene_name": "Peroxisomal membrane protein PEX14",
  "gene": "UniProtKB:O75381",
  "term_id": "GO:0005102"
}